signaling receptor complex adaptor activity [GO:0030159] (molecular function) Definition: The binding activity of a molecule that provides a physical support for the assembly of a multiprotein receptor signaling complex. Sources: GOC:mah Also known as: receptor signaling complex adaptor activity, receptor signaling complex scaffold activity, receptor signaling complex scaffold protein activity, receptor signalling complex adaptor activity, receptor signalling complex scaffold activity Relationships: is a type of GO:0035591; has part signaling receptor binding [GO:0005102] Subtypes: transmembrane receptor protein tyrosine kinase adaptor activity [GO:0005068], synaptic receptor adaptor activity [GO:0030160]